{
  "term_label": "Unknown biological process",
  "term_id": "UNKNOWN:0002",
  "gene_name": "Putative uncharacterized protein encoded by LINC00312",
  "gene": "UniProtKB:Q9Y6C7",
  "gene_symbol": "LINC00312"
}